{
  "gene_symbol": "ATP4B",
  "gene": "UniProtKB:P51164",
  "term_label": "ATPase activator activity",
  "term_id": "GO:0001671",
  "gene_name": "Potassium-transporting ATPase subunit beta"
}